methyl accepting chemotaxis protein complex [GO:0098561] (CC) Note: A number of complexes of this class are found in E.coli. Relationships: is_a protein-containing complex [GO:0032991] Definition: A transmembrane protein complex that consists of multiple methyl-accepting chemoreceptor protein subunits, a histidine kinase and a connector protein and which functions in the regulation of flagellar rotary motor activity in response to an external chemical stimulus. References: PMID:1326408, PMID:15802240 Sources: GOC:dos